{
  "term_label": "Unknown cellular component",
  "gene": "UniProtKB:Q3MIP1",
  "term_id": "UNKNOWN:0003",
  "gene_symbol": "ITPRIPL2",
  "gene_name": "Inositol 1,4,5-trisphosphate receptor-interacting protein-like 2"
}